formamidase activity [GO:0004328] (molecular function) Definition: Catalysis of the reaction: formamide + H2O = formate + NH4. Also known as: formamide hydrolase activity, formamide amidohydrolase activity Sources: RHEA:21948 Relationships: is a type of amidase activity [GO:0004040]